{
  "term_id": "GO:0005634",
  "gene_symbol": "USP28",
  "term_label": "nucleus",
  "gene": "UniProtKB:Q96RU2",
  "gene_name": "Ubiquitin carboxyl-terminal hydrolase 28"
}